cerebral blood circulation [GO:0120275] (biological process) Relationships: is a type of GO:0008015 Also known as: cerebrum blood circulation, telencephelon blood circulation Regulation: regulated by regulation of cerebral blood circulation [GO:0120276]; positively regulated by positive regulation of cerebral blood circulation [GO:0120277]; negatively regulated by GO:0120278 Definition: The flow of blood through the network of arteries and veins supplying the cerebrum, enabling the transport of nutrients to the tissues and the removal of waste products. References: PMID:25397684 Sources: GOC:krc